glucosyl-DNA beta-glucosyltransferase activity [GO:0033822] (molecular function) Sources: EC:2.4.1.28 Definition: Catalysis of the transfer of a beta-D-glucosyl residue from UDP-glucose to a glucosylhydroxymethylcytosine residue in DNA. Relationships: is a type of glucosyltransferase activity [GO:0046527] Also known as: T6-beta-glucosyl transferase activity, T6-glucosyl-HMC-beta-glucosyl transferase activity, UDP-glucose:D-glucosyl-DNA beta-D-glucosyltransferase activity, UDPglucose:D-glucosyl-DNA beta-D-glucosyltransferase activity, uridine diphosphoglucose-glucosyldeoxyribonucleate beta-glucosyltransferase activity